bract morphogenesis [GO:0010433] (biological process) Relationships: is a type of plant organ morphogenesis [GO:1905392]; BFO_0000050 bract development [GO:0010432] Definition: The process in which the anatomical structure of a bract are generated and organized. A bract is a leaf, usually different in form from the foliage leaves, subtending a flower or inflorescence. References: PMID:16554366 Sources: GOC:tb, PO:0009055